fungal-type cell wall organization [GO:0031505] (biological process) Relationships: is a type of cell wall organization [GO:0071555]; is a type of fungal-type cell wall organization or biogenesis [GO:0071852] Sources: GOC:dph, GOC:jl, GOC:mah, GOC:mtg_sensu Definition: A process that is carried out at the cellular level which results in the assembly, arrangement of constituent parts, or disassembly of the fungal-type cell wall. Subtypes: fungal-type cell wall disassembly [GO:0071853], fungal-type cell wall assembly [GO:0071940] Regulation: regulated by regulation of fungal-type cell wall organization [GO:0060237] Also known as: chitin- and beta-glucan-containing cell wall organisation, chitin- and beta-glucan-containing cell wall organization and biogenesis, beta-glucan-containing cell wall organization and biogenesis, chitin-containing cell wall organization and biogenesis, fungal-type cell wall organization and biogenesis